{
  "gene_symbol": "COL6A1",
  "gene": "UniProtKB:P12109",
  "term_id": "GO:0031012",
  "term_label": "extracellular matrix",
  "gene_name": "Collagen alpha-1(VI) chain"
}